RNA polymerase II C-terminal domain S7 O-GlcNAc transferase activity [GO:0140843] (molecular function) Definition: Catalysis of the reaction: UDP-N-acetyl-D-glucosamine + RNA polymerase II large subunit CTD heptapeptide repeat (YSPTSPS) = UDP + RNA polymerase II large subunit CTD heptapeptide repeat 3-O-(N-acetyl-D-glucosaminyl)-L-serine (position 7). Relationships: is a type of RNA polymerase II C-terminal domain O-GlcNAc transferase activity [GO:0140841] References: PMID:22605332